{
  "term_label": "protein serine/threonine kinase activity",
  "gene_symbol": "MAPK15",
  "term_id": "GO:0004674",
  "gene": "UniProtKB:Q8TD08",
  "gene_name": "Mitogen-activated protein kinase 15"
}